{
  "gene_name": "Neurotrophin-4",
  "term_id": "GO:0005615",
  "gene_symbol": "NTF4",
  "gene": "UniProtKB:P34130",
  "term_label": "extracellular space"
}